interleukin-4 binding [GO:0019979] (molecular function) Definition: Binding to interleukin-4. Sources: GOC:jl Also known as: IL-4 binding Relationships: is a type of growth factor binding [GO:0019838]; is_a cytokine binding [GO:0019955]